regulation of cell proliferation involved in compound eye morphogenesis [GO:2000495] (biological process) Definition: Any process that modulates the frequency, rate or extent of cell proliferation involved in compound eye morphogenesis. Sources: GOC:obol Subtypes: negative regulation of cell proliferation involved in compound eye morphogenesis [GO:2000496], positive regulation of cell proliferation involved in compound eye morphogenesis [GO:2000497] Relationships: is a type of regulation of cell population proliferation [GO:0042127]; regulates cell proliferation involved in compound eye morphogenesis [GO:0035736]